{
  "gene_name": "DDB1- and CUL4-associated factor 4-like protein 2",
  "term_id": "UNKNOWN:0002",
  "gene_symbol": "DCAF4L2",
  "term_label": "Unknown biological process",
  "gene": "UniProtKB:Q8NA75"
}